{
  "gene": "UniProtKB:Q6L8G4",
  "gene_symbol": "KRTAP5-11",
  "term_label": "Unknown biological process",
  "term_id": "UNKNOWN:0002",
  "gene_name": "Keratin-associated protein 5-11"
}